{
  "gene": "UniProtKB:Q8WUJ3",
  "term_label": "Unknown molecular function",
  "gene_name": "Cell migration-inducing and hyaluronan-binding protein",
  "gene_symbol": "CEMIP",
  "term_id": "UNKNOWN:0001"
}